{
  "gene": "UniProtKB:Q9H2A3",
  "gene_symbol": "NEUROG2",
  "gene_name": "Neurogenin-2",
  "term_label": "sensory organ development",
  "term_id": "GO:0007423"
}